{
  "gene_symbol": "AJAP1",
  "term_id": "UNKNOWN:0002",
  "gene_name": "Adherens junction-associated protein 1",
  "term_label": "Unknown biological process",
  "gene": "UniProtKB:Q9UKB5"
}